{
  "gene": "UniProtKB:Q9P2V4",
  "gene_name": "Leucine-rich repeat, immunoglobulin-like domain and transmembrane domain-containing protein 1",
  "term_label": "endoplasmic reticulum membrane",
  "gene_symbol": "LRIT1",
  "term_id": "GO:0005789"
}